{
  "gene": "UniProtKB:Q8IV50",
  "gene_name": "LysM and putative peptidoglycan-binding domain-containing protein 2",
  "term_label": "Unknown biological process",
  "gene_symbol": "LYSMD2",
  "term_id": "UNKNOWN:0002"
}